{
  "gene": "UniProtKB:P22626",
  "gene_symbol": "HNRNPA2B1",
  "term_label": "mRNA splicing, via spliceosome",
  "gene_name": "Heterogeneous nuclear ribonucleoproteins A2_B1",
  "term_id": "GO:0000398"
}